{
  "gene_symbol": "LCA5L",
  "gene": "UniProtKB:O95447",
  "term_label": "axoneme",
  "gene_name": "Lebercilin-like protein",
  "term_id": "GO:0005930"
}